{
  "term_label": "metalloendopeptidase activity",
  "gene_name": "Disintegrin and metalloproteinase domain-containing protein 12",
  "term_id": "GO:0004222",
  "gene_symbol": "ADAM12",
  "gene": "UniProtKB:O43184"
}